{
  "gene": "UniProtKB:Q99928",
  "gene_name": "Gamma-aminobutyric acid receptor subunit gamma-3",
  "term_label": "chloride transmembrane transport",
  "gene_symbol": "GABRG3",
  "term_id": "GO:1902476"
}